{
  "gene": "UniProtKB:Q8NBI3",
  "gene_name": "Draxin",
  "gene_symbol": "DRAXIN",
  "term_id": "GO:0021528",
  "term_label": "commissural neuron differentiation in spinal cord"
}